{
  "term_label": "axon guidance",
  "gene": "UniProtKB:O60469",
  "term_id": "GO:0007411",
  "gene_symbol": "DSCAM",
  "gene_name": "Cell adhesion molecule DSCAM"
}